{
  "gene_symbol": "WASF3",
  "term_label": "protein kinase A regulatory subunit binding",
  "term_id": "GO:0034237",
  "gene_name": "Actin-binding protein WASF3",
  "gene": "UniProtKB:Q9UPY6"
}